{
  "term_label": "(3R)-hydroxyacyl-[acyl-carrier-protein] dehydratase activity",
  "gene_symbol": "HTD2",
  "gene_name": "Hydroxyacyl-thioester dehydratase type 2, mitochondrial",
  "term_id": "GO:0019171",
  "gene": "UniProtKB:P86397"
}